{
  "gene_name": "Serine_threonine-protein kinase_endoribonuclease IRE1",
  "term_id": "GO:0051082",
  "term_label": "unfolded protein binding",
  "gene": "UniProtKB:O75460",
  "gene_symbol": "ERN1"
}